{
  "gene_symbol": "SYNGAP1",
  "gene": "UniProtKB:Q96PV0",
  "term_id": "UNKNOWN:0003",
  "gene_name": "Ras_Rap GTPase-activating protein SynGAP",
  "term_label": "Unknown cellular component"
}